{
  "term_label": "Unknown molecular function",
  "term_id": "UNKNOWN:0001",
  "gene_symbol": "CREBZF",
  "gene": "UniProtKB:Q9NS37",
  "gene_name": "CREB_ATF bZIP transcription factor"
}